{
  "term_id": "GO:0042552",
  "gene_name": "Myelin protein P0",
  "gene": "UniProtKB:P25189",
  "gene_symbol": "MPZ",
  "term_label": "myelination"
}